{
  "gene_symbol": "ZFP36",
  "gene": "UniProtKB:P26651",
  "term_label": "protein-RNA sequence-specific adaptor activity",
  "gene_name": "mRNA decay activator protein ZFP36",
  "term_id": "GO:0160134"
}